{
  "term_label": "Unknown molecular function",
  "gene": "UniProtKB:Q8N9U9",
  "gene_name": "Putative uncharacterized protein SPANXA2-OT1",
  "term_id": "UNKNOWN:0001",
  "gene_symbol": "SPANXA2-OT1"
}